sperm glycocalyx [GO:0120238] (cellular component) Definition: The carbohydrate rich layer at the outermost periphery of a sperm cell. Relationships: is a type of glycocalyx [GO:0030112] Sources: GOC:krc